{
  "gene_name": "Uncharacterized protein C8orf74",
  "term_label": "Unknown cellular component",
  "gene_symbol": "C8orf74",
  "term_id": "UNKNOWN:0003",
  "gene": "UniProtKB:Q6P047"
}